{
  "gene_name": "E1A-binding protein p400",
  "gene": "UniProtKB:Q96L91",
  "term_label": "NuA4 histone acetyltransferase complex",
  "gene_symbol": "EP400",
  "term_id": "GO:0035267"
}